aconitate decarboxylase activity [GO:0047613] (molecular function) Also known as: CAD activity, cis-aconitate carboxy-lyase (itaconate-forming), cis-aconitate carboxy-lyase activity, cis-aconitic decarboxylase activity Relationships: is a type of carboxy-lyase activity [GO:0016831] Sources: EC:4.1.1.6, RHEA:15253 Definition: Catalysis of the reaction: cis-aconitate + H+ = CO2 + itaconate.